{
  "term_id": "UNKNOWN:0003",
  "gene_name": "Testis-specific serine_threonine-protein kinase 3",
  "term_label": "Unknown cellular component",
  "gene_symbol": "TSSK3",
  "gene": "UniProtKB:Q96PN8"
}